{
  "gene_name": "Zinc finger protein 821",
  "gene_symbol": "ZNF821",
  "term_id": "UNKNOWN:0003",
  "term_label": "Unknown cellular component",
  "gene": "UniProtKB:O75541"
}